establishment of synaptic vesicle localization [GO:0097480] (biological process) Also known as: establishment of synaptic vesicle localisation Sources: GOC:pr Definition: The directed movement of a synaptic vesicle or vesicles to a specific location. Relationships: is a type of GO:0051650; is part of GO:0097479